{
  "term_label": "cytosol",
  "term_id": "GO:0005829",
  "gene_name": "B-cell lymphoma_leukemia 10",
  "gene": "UniProtKB:O95999",
  "gene_symbol": "BCL10"
}